{
  "gene_symbol": "DAXX",
  "term_id": "GO:0005634",
  "gene_name": "Death domain-associated protein 6",
  "term_label": "nucleus",
  "gene": "UniProtKB:Q9UER7"
}